{
  "term_id": "GO:0030099",
  "gene_symbol": "TET2",
  "gene": "UniProtKB:Q6N021",
  "term_label": "myeloid cell differentiation",
  "gene_name": "Methylcytosine dioxygenase TET2"
}